callose localization [GO:0052545] (biological process) Also known as: callose localisation References: PMID:18397379 Sources: GOC:mtg_pamgo_17jul06 Definition: Any process in which callose is transported to, and/or maintained in, a specific location. Callose is a linear 1,3-beta-d-glucan formed from UDP-glucose and is found in certain plant cell walls. Relationships: is a type of polysaccharide localization [GO:0033037] Subtypes: GO:0052542, callose deposition in cell wall [GO:0052543], callose deposition in phloem sieve plate [GO:0080165]